{
  "gene_name": "Interleukin-2",
  "term_id": "GO:0005615",
  "term_label": "extracellular space",
  "gene_symbol": "IL2",
  "gene": "UniProtKB:P60568"
}